{
  "gene": "UniProtKB:Q9UKW4",
  "gene_symbol": "VAV3",
  "term_label": "cytoplasm",
  "term_id": "GO:0005737",
  "gene_name": "Guanine nucleotide exchange factor VAV3"
}